{
  "gene_symbol": "CCDC88C",
  "term_id": "GO:0008017",
  "gene_name": "Protein Daple",
  "gene": "UniProtKB:Q9P219",
  "term_label": "microtubule binding"
}